{
  "term_label": "plasma membrane",
  "gene_name": "Sodium_hydrogen exchanger 5",
  "term_id": "GO:0005886",
  "gene": "UniProtKB:Q14940",
  "gene_symbol": "SLC9A5"
}